dolichyldiphosphatase activity [GO:0047874] (molecular function) Definition: Catalysis of the reaction: a di-trans,poly-cis-dolichyl diphosphate + H2O = a di-trans,poly-cis-dolichyl phosphate + phosphate + H+. Sources: RHEA:14385 Also known as: dolichol diphosphatase activity, dolichyl diphosphate phosphohydrolase activity, dolichyl pyrophosphatase activity, dolichyl-diphosphate phosphohydrolase activity Relationships: is a type of polyprenyl diphosphate phosphatase activity [GO:0120556]